dimethylsilanediol metabolic process [GO:0046454] (biological process) Also known as: dimethylsilanediol metabolism Definition: The chemical reactions and pathways involving dimethylsilanediol, the smallest member of the dialkylsilanediols. Dimethylsilanediol is the monomer of polydimethylsiloxane, a compound which can be found in a wide range of industrial and consumer products. Subtypes: GO:0042210 Sources: GOC:ai Relationships: is a type of small molecule metabolic process [GO:0044281]